{
  "gene_name": "FYVE, RhoGEF and PH domain-containing protein 4",
  "gene": "UniProtKB:Q96M96",
  "gene_symbol": "FGD4",
  "term_id": "GO:0007010",
  "term_label": "cytoskeleton organization"
}